{
  "gene": "UniProtKB:A6NGN9",
  "term_id": "UNKNOWN:0001",
  "term_label": "Unknown molecular function",
  "gene_name": "IgLON family member 5",
  "gene_symbol": "IGLON5"
}